{
  "term_id": "GO:0031267",
  "gene": "UniProtKB:Q9UJY4",
  "gene_name": "ADP-ribosylation factor-binding protein GGA2",
  "term_label": "small GTPase binding",
  "gene_symbol": "GGA2"
}